{
  "gene_name": "Protein PET100 homolog, mitochondrial",
  "term_id": "GO:0033617",
  "gene": "UniProtKB:P0DJ07",
  "gene_symbol": "PET100",
  "term_label": "mitochondrial respiratory chain complex IV assembly"
}